{
  "gene_symbol": "CACNA1B",
  "term_id": "GO:0007268",
  "gene_name": "Voltage-dependent N-type calcium channel subunit alpha-1B",
  "term_label": "chemical synaptic transmission",
  "gene": "UniProtKB:Q00975"
}